{
  "gene_symbol": "ZNF572",
  "gene": "UniProtKB:Q7Z3I7",
  "term_label": "nucleoplasm",
  "term_id": "GO:0005654",
  "gene_name": "Zinc finger protein 572"
}